hindbrain structural organization [GO:0021577] (biological process) Definition: The process that contributes to the act of creating the structural organization of the hindbrain. This process pertains to the physical shaping of a rudimentary structure. The hindbrain is the region consisting of the medulla, pons and cerebellum. Areas of the hindbrain control motor and autonomic functions. Relationships: is a type of GO:0048532; is part of hindbrain morphogenesis [GO:0021575] Sources: GOC:cls, GOC:dgh, GOC:dph, GOC:jid, GO_REF:0000021 Also known as: hindbrain structural organisation